{
  "gene_name": "Electron transfer flavoprotein subunit alpha, mitochondrial",
  "term_id": "GO:0050660",
  "term_label": "flavin adenine dinucleotide binding",
  "gene_symbol": "ETFA",
  "gene": "UniProtKB:P13804"
}